germ-line stem-cell niche homeostasis [GO:0060250] (biological process) Sources: GOC:dph Definition: A homeostatic process involved in the maintenance of an internal steady state within the germ-line stem-cell niche. This includes control of cellular proliferation and death and control of metabolic function that allows the niche to continue to function. A gem-line stem-cell niche is an anatomical structure that regulates how germ-line stem-cells are used and saves them from depletion. Also known as: germ-line stem-cell niche maintenance, maintenance of germ line stem cell niche, maintenance of germ line stem-cell niche, maintenance of germ-line stem cell niche, maintenance of germ-line stem-cell niche Relationships: is a type of anatomical structure homeostasis [GO:0060249]